{
  "gene": "UniProtKB:A0A2R8YED5",
  "term_id": "GO:0005549",
  "gene_symbol": "OR5BS1",
  "gene_name": "Olfactory receptor",
  "term_label": "odorant binding"
}